{
  "gene_symbol": "PIWIL2",
  "term_label": "nucleus",
  "gene": "UniProtKB:Q8TC59",
  "term_id": "GO:0005634",
  "gene_name": "Piwi-like protein 2"
}